{
  "term_label": "Unknown molecular function",
  "gene": "UniProtKB:A4D1U4",
  "term_id": "UNKNOWN:0001",
  "gene_name": "DENN domain-containing protein 11",
  "gene_symbol": "DENND11"
}